{
  "term_id": "GO:0071819",
  "gene": "UniProtKB:Q14CW9",
  "gene_name": "Ataxin-7-like protein 3",
  "term_label": "DUBm complex",
  "gene_symbol": "ATXN7L3"
}